{
  "term_label": "olfactory receptor activity",
  "term_id": "GO:0004984",
  "gene_symbol": "OR4F17",
  "gene_name": "Olfactory receptor 4F17",
  "gene": "UniProtKB:Q8NGA8"
}